{
  "term_id": "GO:0035556",
  "gene_symbol": "STK38",
  "gene": "UniProtKB:Q15208",
  "gene_name": "Serine_threonine-protein kinase 38",
  "term_label": "intracellular signal transduction"
}